{
  "gene_name": "BPI fold-containing family A member 2",
  "gene_symbol": "BPIFA2",
  "term_id": "GO:0030141",
  "gene": "UniProtKB:Q96DR5",
  "term_label": "secretory granule"
}